establishment or maintenance of actin cytoskeleton polarity [GO:0030950] (biological process) Relationships: is a type of actin cytoskeleton organization [GO:0030036]; is a type of establishment or maintenance of cytoskeleton polarity [GO:0030952] Definition: Any cellular process that results in the specification, formation or maintenance of polarized actin-based cytoskeletal structures. Sources: GOC:mah